{
  "gene": "UniProtKB:Q15560",
  "gene_name": "Transcription elongation factor A protein 2",
  "term_id": "GO:0003711",
  "term_label": "transcription elongation factor activity",
  "gene_symbol": "TCEA2"
}